{
  "gene_name": "Homeobox protein Hox-D11",
  "term_id": "GO:0005634",
  "gene_symbol": "HOXD11",
  "gene": "UniProtKB:P31277",
  "term_label": "nucleus"
}